{
  "gene_symbol": "ADGRE3",
  "term_label": "G protein-coupled receptor signaling pathway",
  "gene_name": "Adhesion G protein-coupled receptor E3",
  "gene": "UniProtKB:Q9BY15",
  "term_id": "GO:0007186"
}